{
  "gene_symbol": "IGLV2-8",
  "gene": "UniProtKB:P01709",
  "gene_name": "Immunoglobulin lambda variable 2-8",
  "term_id": "GO:0019814",
  "term_label": "immunoglobulin complex"
}